{
  "gene": "UniProtKB:Q8NGE7",
  "gene_name": "Olfactory receptor 9K2",
  "term_label": "olfactory receptor activity",
  "term_id": "GO:0004984",
  "gene_symbol": "OR9K2"
}